{
  "gene": "UniProtKB:O15164",
  "gene_symbol": "TRIM24",
  "term_label": "Unknown biological process",
  "gene_name": "Transcription intermediary factor 1-alpha",
  "term_id": "UNKNOWN:0002"
}